{
  "term_label": "Unknown molecular function",
  "gene_symbol": "HAO1",
  "gene_name": "2-Hydroxyacid oxidase 1",
  "gene": "UniProtKB:Q9UJM8",
  "term_id": "UNKNOWN:0001"
}